{
  "gene_name": "Proenkephalin-A",
  "term_id": "GO:0005886",
  "gene_symbol": "PENK",
  "gene": "UniProtKB:P01210",
  "term_label": "plasma membrane"
}